{
  "gene_symbol": "SESTD1",
  "term_label": "phosphatidylinositol-4-phosphate binding",
  "term_id": "GO:0070273",
  "gene_name": "SEC14 domain and spectrin repeat-containing protein 1",
  "gene": "UniProtKB:Q86VW0"
}